{
  "gene": "UniProtKB:Q96MG8",
  "gene_symbol": "PCMTD1",
  "term_label": "cytoplasm",
  "term_id": "GO:0005737",
  "gene_name": "Protein-L-isoaspartate O-methyltransferase domain-containing protein 1"
}